{
  "gene_symbol": "FTH1",
  "gene": "UniProtKB:P02794",
  "gene_name": "Ferritin heavy chain",
  "term_label": "ferrous iron binding",
  "term_id": "GO:0008198"
}